{
  "gene": "UniProtKB:Q8NH95",
  "gene_name": "Putative olfactory receptor 13C6",
  "term_id": "GO:0005886",
  "gene_symbol": "OR13C6P",
  "term_label": "plasma membrane"
}